anatomical structure arrangement [GO:0048532] (biological process) Subtypes: optic cup structural organization [GO:0003409], meristem structural organization [GO:0009933], GO:0010358, midbrain-hindbrain boundary structural organization [GO:0021552], hindbrain structural organization [GO:0021577], GO:0021581, pons structural organization [GO:0021585], GO:0021589, rhombomere structural organization [GO:0021595], GO:0021597, cranial nerve structural organization [GO:0021604], cerebellar granular layer structural organization [GO:0021685], cerebellar molecular layer structural organization [GO:0021689], GO:0021693, cerebellar cortex structural organization [GO:0021698], inferior olivary nucleus structural organization [GO:0021716], GO:0021721, dorsal motor nucleus of vagus nerve structural organization [GO:0035763], mesoderm structural organization [GO:0048338], floral organ structural organization [GO:0048450], floral whorl structural organization [GO:0048459], flower structural organization [GO:0048461], outer ear unfolding [GO:0060185], ganglion structural organization [GO:0061555], pronephros structural organization [GO:0072118], quiescent center organization [GO:1904961] Definition: The process that gives rise to the configuration of the constituent parts of an anatomical structure. This process pertains to the physical shaping of a rudimentary structure. Anatomical structures can be macroscopic such as a carpel, or microscopic such as an acrosome. Sources: GOC:go_curators Also known as: anatomical structure organization, anatomical structure structural organization, organization of an anatomical structure, structural organization Relationships: is a type of GO:0032502; is part of anatomical structure morphogenesis [GO:0009653]